maltose phosphorylase activity [GO:0050082] (molecular function) Also known as: maltose:phosphate 1-beta-D-glucosyltransferase activity Relationships: is a type of 1,4-alpha-oligoglucan phosphorylase activity [GO:0004645] Definition: Catalysis of the reaction: maltose + phosphate = D-glucose + beta-D-glucose 1-phosphate. Sources: EC:2.4.1.8, MetaCyc:MALTOSE-PHOSPHORYLASE-RXN